{
  "gene_name": "Dehydrogenase_reductase SDR family member 7C",
  "gene": "UniProtKB:A6NNS2",
  "term_id": "GO:0016616",
  "term_label": "oxidoreductase activity, acting on the CH-OH group of donors, NAD or NADP as acceptor",
  "gene_symbol": "DHRS7C"
}